hydroxyproline transport [GO:0034589] (biological process) References: PMID:14502423 Sources: GOC:mah Also known as: 4-hydroxyproline transport, L-hydroxyproline transport Definition: The directed movement of hydroxyproline into, out of or within a cell, or between cells, by means of some agent such as a transporter or pore. Relationships: is a type of amino acid transport [GO:0006865]; is a type of carboxylic acid transport [GO:0046942]; is a type of modified amino acid transport [GO:0072337]